{
  "gene_symbol": "GIMD1",
  "gene": "UniProtKB:P0DJR0",
  "term_label": "Unknown cellular component",
  "gene_name": "GTPase IMAP family member GIMD1",
  "term_id": "UNKNOWN:0003"
}